{
  "gene_name": "Keratin-associated protein 13-3",
  "term_label": "Unknown molecular function",
  "gene": "UniProtKB:Q3SY46",
  "gene_symbol": "KRTAP13-3",
  "term_id": "UNKNOWN:0001"
}